{
  "gene_name": "Dynein axonemal heavy chain 8",
  "gene_symbol": "DNAH8",
  "gene": "UniProtKB:Q96JB1",
  "term_id": "GO:0051959",
  "term_label": "dynein light intermediate chain binding"
}